optic vesicle formation [GO:0003403] (BP) Definition: The developmental process pertaining to the initial formation of the optic vesicle from the lateral wall of the forebrain. This process begins with the specific processes that contribute to the appearance of the vesicle and ends when the vesicle has evaginated. The optic vesicle is the evagination of neurectoderm that precedes formation of the optic cup. Sources: GOC:ascb_2009, GOC:dph, GOC:tb Relationships: is a type of anatomical structure formation involved in morphogenesis [GO:0048646]; BFO_0000050 optic vesicle morphogenesis [GO:0003404]; is part of embryonic camera-type eye formation [GO:0060900]